{
  "gene_symbol": "TBCD",
  "term_id": "GO:0006457",
  "term_label": "protein folding",
  "gene": "UniProtKB:Q9BTW9",
  "gene_name": "Tubulin-specific chaperone D"
}